{
  "term_label": "translation",
  "term_id": "GO:0006412",
  "gene": "UniProtKB:P82675",
  "gene_name": "Small ribosomal subunit protein uS5m",
  "gene_symbol": "MRPS5"
}